{
  "term_id": "GO:1905515",
  "gene": "UniProtKB:Q96NH3",
  "term_label": "non-motile cilium assembly",
  "gene_name": "Protein broad-minded",
  "gene_symbol": "TBC1D32"
}